{
  "term_id": "GO:0005911",
  "gene_symbol": "CASK",
  "gene_name": "Peripheral plasma membrane protein CASK",
  "term_label": "cell-cell junction",
  "gene": "UniProtKB:O14936"
}